{
  "gene": "UniProtKB:Q6A163",
  "gene_name": "Keratin, type I cytoskeletal 39",
  "term_label": "intermediate filament organization",
  "gene_symbol": "KRT39",
  "term_id": "GO:0045109"
}